ATP export [GO:1904669] (biological process) Also known as: ATP efflux References: PMID:24286344 Sources: GOC:TermGenie, GO_REF:0000074 Definition: The directed movement of ATP out of a cell or organelle. Relationships: is a type of ATP transport [GO:0015867]